{
  "gene": "UniProtKB:P26678",
  "term_id": "GO:0010459",
  "gene_symbol": "PLN",
  "gene_name": "Cardiac phospholamban",
  "term_label": "negative regulation of heart rate"
}